{
  "gene_name": "LIM domain-containing protein ajuba",
  "gene": "UniProtKB:Q96IF1",
  "gene_symbol": "AJUBA",
  "term_label": "regulation of DNA-templated transcription",
  "term_id": "GO:0006355"
}